dITP diphosphatase activity [GO:0035870] (molecular function) References: PMID:21548881 Sources: GOC:dgf, RHEA:28342 Definition: Catalysis of the reaction: dITP + H2O = dIMP + H+ + diphosphate. Relationships: is_a nucleoside triphosphate diphosphatase activity [GO:0047429] Also known as: 2'-deoxyinosine-5'-triphosphate pyrophosphohydrolase activity, dITP pyrophosphatase activity, deoxyinosine triphosphate pyrophosphatase activity